regulation of norepinephrine uptake [GO:0051621] (biological process) Subtypes: negative regulation of norepinephrine uptake [GO:0051622], positive regulation of norepinephrine uptake [GO:0051623] Definition: Any process that modulates the frequency, rate or extent of the directed movement of the neurotransmitter norepinephrine into a cell. Also known as: regulation of levarterenol uptake, regulation of noradrenaline uptake, regulation of norepinephrine import Relationships: is a type of regulation of transport [GO:0051049]; regulates norepinephrine uptake [GO:0051620] Sources: GOC:ai